plastid chromosome [GO:0009508] (cellular component) Sources: ISBN:0943088399 Relationships: is a type of chromosome [GO:0005694]; is part of plastid nucleoid [GO:0042646] Subtypes: GO:0042648 Definition: A circular DNA molecule containing plastid encoded genes.